{
  "term_label": "nucleus",
  "gene_symbol": "TNFAIP3",
  "term_id": "GO:0005634",
  "gene": "UniProtKB:P21580",
  "gene_name": "Tumor necrosis factor alpha-induced protein 3"
}